{
  "term_id": "GO:0006954",
  "term_label": "inflammatory response",
  "gene_symbol": "PTGIR",
  "gene_name": "Prostacyclin receptor",
  "gene": "UniProtKB:P43119"
}